long-term strengthening of neuromuscular junction [GO:0042062] (biological process) Definition: Any process that results in an increase in the efficacy of transmission at a neuromuscular synapse. Relationships: is a type of GO:0050806; is part of regulation of synaptic assembly at neuromuscular junction [GO:0008582] Sources: GO_REF:0000021